collenchyma cell differentiation [GO:0048761] (biological process) Sources: CL:0000330, GOC:jid, PO:0000075 Relationships: is a type of GO:0030154 Definition: The process in which a relatively unspecialized cell acquires specialized features of a collenchyma cell. This is a plant cell in which the primary cell walls are unevenly thickened, with most thickening occurring at the cell corners. Cells are living and able to grow, they are elongated, and lignin and secondary walls absent. Collenchyma cells make up collenchyma tissue which acts as a supporting tissue in growing shoots, leaves and petioles. This tissue is often arranged in cortical ribs, as seen prominently in celery and rhubarb petioles.